{
  "gene_symbol": "WASHC2C",
  "gene_name": "WASH complex subunit 2C",
  "term_id": "GO:1905394",
  "gene": "UniProtKB:Q9Y4E1",
  "term_label": "retromer complex binding"
}